{
  "gene_name": "Perilipin-1",
  "term_label": "lipid droplet",
  "term_id": "GO:0005811",
  "gene_symbol": "PLIN1",
  "gene": "UniProtKB:O60240"
}